{
  "gene": "UniProtKB:Q8NGJ9",
  "gene_symbol": "OR51T1",
  "term_label": "olfactory receptor activity",
  "gene_name": "Olfactory receptor 51T1",
  "term_id": "GO:0004984"
}